{
  "gene_name": "Zinc finger Y-chromosomal protein",
  "gene_symbol": "ZFY",
  "term_label": "sequence-specific DNA binding",
  "gene": "UniProtKB:P08048",
  "term_id": "GO:0043565"
}